female genitalia development [GO:0030540] (BP) Definition: The process whose specific outcome is the progression of the female genitalia over time, from formation to the mature structure. Sources: GOC:mah Also known as: female genital development Relationships: is a type of GO:0048806; is part of female sex differentiation [GO:0046660] Subtypes: imaginal disc-derived female genitalia development [GO:0007486], GO:0060068